{
  "gene_symbol": "CHST5",
  "term_label": "sulfur compound metabolic process",
  "gene_name": "Carbohydrate sulfotransferase 5",
  "gene": "UniProtKB:Q9GZS9",
  "term_id": "GO:0006790"
}